{
  "gene_name": "Uncharacterized protein",
  "term_id": "UNKNOWN:0001",
  "gene_symbol": "A0A8I5KPI3",
  "gene": "UniProtKB:A0A8I5KPI3",
  "term_label": "Unknown molecular function"
}